positive regulation of histamine uptake [GO:0051618] (biological process) Sources: GOC:ai Also known as: positive regulation of histamine import, up regulation of histamine uptake, up-regulation of histamine uptake, upregulation of histamine uptake, activation of histamine uptake, stimulation of histamine uptake Relationships: is a type of positive regulation of neurotransmitter uptake [GO:0051582]; is a type of regulation of histamine uptake [GO:0051616]; positively regulates histamine uptake [GO:0051615] Definition: Any process that activates or increases the frequency, rate or extent of the directed movement of histamine into a cell.